{
  "term_id": "GO:0050930",
  "gene_name": "Stromal cell-derived factor 1",
  "gene": "UniProtKB:P48061",
  "term_label": "induction of positive chemotaxis",
  "gene_symbol": "CXCL12"
}